{
  "gene": "UniProtKB:D6RGX4",
  "term_id": "UNKNOWN:0003",
  "gene_symbol": "FAM90A26",
  "term_label": "Unknown cellular component",
  "gene_name": "Putative protein FAM90A26"
}